{
  "gene_name": "Voltage-dependent L-type calcium channel subunit alpha-1F",
  "gene_symbol": "CACNA1F",
  "gene": "UniProtKB:O60840",
  "term_id": "GO:0098703",
  "term_label": "calcium ion import across plasma membrane"
}